{
  "term_label": "sperm flagellum",
  "gene_name": "Tektin-4",
  "gene": "UniProtKB:Q8WW24",
  "term_id": "GO:0036126",
  "gene_symbol": "TEKT4"
}